{
  "gene_symbol": "NRIP2",
  "gene_name": "Nuclear receptor-interacting protein 2",
  "gene": "UniProtKB:Q9BQI9",
  "term_label": "cytoplasm",
  "term_id": "GO:0005737"
}